{
  "gene_name": "Choline_ethanolaminephosphotransferase 1",
  "gene": "UniProtKB:Q9Y6K0",
  "term_label": "phosphatidylethanolamine biosynthetic process",
  "term_id": "GO:0006646",
  "gene_symbol": "CEPT1"
}